{
  "gene": "UniProtKB:Q6ZYL4",
  "term_label": "Unknown molecular function",
  "gene_symbol": "GTF2H5",
  "term_id": "UNKNOWN:0001",
  "gene_name": "General transcription factor IIH subunit 5"
}